{
  "gene_name": "C-X-C chemokine receptor type 2",
  "gene": "UniProtKB:P25025",
  "term_id": "GO:0016493",
  "term_label": "C-C chemokine receptor activity",
  "gene_symbol": "CXCR2"
}